{
  "term_label": "cytoskeleton",
  "gene": "UniProtKB:A8K5M9",
  "term_id": "GO:0005856",
  "gene_symbol": "C15orf62",
  "gene_name": "Uncharacterized protein C15orf62, mitochondrial"
}